{
  "gene": "UniProtKB:P52569",
  "gene_name": "Cationic amino acid transporter 2",
  "gene_symbol": "SLC7A2",
  "term_id": "GO:0097638",
  "term_label": "L-arginine import across plasma membrane"
}